VRK3/VHR/ERK complex [GO:0002167] (cellular component) Definition: A ternary complex consisting of VRK3, VHR (Dusp3), and ERK1 (Mapk3) existing in neuronal cells, and is involved in regulation of the ERK signaling pathway. References: PMID:16845380 Sources: GOC:hjd Relationships: is a type of GO:0032991